regulation of primary metabolic process [GO:0080090] (BP) Relationships: is a type of regulation of metabolic process [GO:0019222]; regulates primary metabolic process [GO:0044238] Subtypes: regulation of carbohydrate metabolic process [GO:0006109], regulation of amino acid metabolic process [GO:0006521], regulation of flavonoid biosynthetic process [GO:0009962], GO:0010967, GO:0019216, GO:0019219, regulation of anthocyanin metabolic process [GO:0031537], regulation of catecholamine metabolic process [GO:0042069], regulation of RNA splicing [GO:0043484], regulation of protein metabolic process [GO:0051246], regulation of acetylcholine metabolic process [GO:0060408], regulation of regulatory ncRNA processing [GO:0070920] References: PMID:19211694 Definition: Any process that modulates the frequency, rate or extent of the chemical reactions and pathways within a cell or an organism involving those compounds formed as a part of the normal anabolic and catabolic processes. These processes take place in most, if not all, cells of the organism.